{
  "term_label": "Unknown molecular function",
  "gene_symbol": "R3HDM4",
  "gene": "UniProtKB:Q96D70",
  "term_id": "UNKNOWN:0001",
  "gene_name": "R3H domain-containing protein 4"
}